{
  "term_label": "Unknown cellular component",
  "gene": "UniProtKB:Q96HM7",
  "term_id": "UNKNOWN:0003",
  "gene_symbol": "PCED1B",
  "gene_name": "PC-esterase domain-containing protein 1B"
}